{
  "term_label": "GTPase activity",
  "gene": "UniProtKB:Q7Z6P3",
  "gene_name": "Ras-related protein Rab-44",
  "term_id": "GO:0003924",
  "gene_symbol": "RAB44"
}